{
  "term_id": "GO:0005740",
  "gene": "UniProtKB:Q14318",
  "gene_symbol": "FKBP8",
  "term_label": "mitochondrial envelope",
  "gene_name": "Peptidyl-prolyl cis-trans isomerase FKBP8"
}